{
  "gene_symbol": "RAD9A",
  "term_id": "GO:0000076",
  "term_label": "DNA replication checkpoint signaling",
  "gene": "UniProtKB:Q99638",
  "gene_name": "Cell cycle checkpoint control protein RAD9A"
}